negative regulation of smooth muscle cell chemotaxis [GO:0071672] (biological process) Definition: Any process that stops, prevents, or reduces the frequency, rate, or extent of smooth muscle cell chemotaxis. Sources: GOC:mah Also known as: down regulation of smooth muscle cell chemotaxis, down-regulation of smooth muscle cell chemotaxis, downregulation of smooth muscle cell chemotaxis, inhibition of smooth muscle cell chemotaxis Relationships: is a type of negative regulation of smooth muscle cell migration [GO:0014912]; is a type of negative regulation of chemotaxis [GO:0050922]; is a type of regulation of smooth muscle cell chemotaxis [GO:0071671]; negatively regulates smooth muscle cell chemotaxis [GO:0071670]